{
  "gene_symbol": "CCR8",
  "term_label": "calcium-mediated signaling",
  "gene_name": "C-C chemokine receptor type 8",
  "gene": "UniProtKB:P51685",
  "term_id": "GO:0019722"
}